forelimb morphogenesis [GO:0035136] (biological process) Sources: GOC:go_curators Definition: The process in which the anatomical structures of the forelimb are generated and organized. The forelimbs are the front limbs of an animal, e.g. the arms of a human. Subtypes: embryonic forelimb morphogenesis [GO:0035115], post-embryonic forelimb morphogenesis [GO:0035128] Relationships: is a type of GO:0035108 Also known as: arm morphogenesis